{
  "gene_symbol": "ANTKMT",
  "term_id": "GO:0016279",
  "gene_name": "Adenine nucleotide translocase lysine N-methyltransferase",
  "term_label": "protein-lysine N-methyltransferase activity",
  "gene": "UniProtKB:Q9BQD7"
}